{
  "term_label": "guanine salvage",
  "term_id": "GO:0006178",
  "gene_symbol": "HPRT1",
  "gene": "UniProtKB:P00492",
  "gene_name": "Hypoxanthine-guanine phosphoribosyltransferase"
}